{
  "term_label": "CENP-A containing chromatin assembly",
  "gene_symbol": "OIP5",
  "term_id": "GO:0034080",
  "gene": "UniProtKB:O43482",
  "gene_name": "Protein Mis18-beta"
}